negative regulation of 1-phosphatidyl-1D-myo-inositol 4,5-bisphosphate biosynthetic process [GO:1902647] (biological process) Definition: Any process that stops, prevents or reduces the frequency, rate or extent of 1-phosphatidyl-1D-myo-inositol 4,5-bisphosphate biosynthetic process. Relationships: is a type of negative regulation of phosphatidylinositol biosynthetic process [GO:0010512]; is a type of regulation of 1-phosphatidyl-1D-myo-inositol 4,5-bisphosphate biosynthetic process [GO:1902646]; negatively regulates 1-phosphatidyl-1D-myo-inositol 4,5-bisphosphate biosynthetic process [GO:1902635] References: PMID:22562153 Sources: GOC:TermGenie, GOC:di, GO_REF:0000058 Also known as: down regulation of 1-phosphatidyl-1D-myo-inositol 4,5-bisphosphate anabolism, down regulation of 1-phosphatidyl-1D-myo-inositol 4,5-bisphosphate biosynthesis, down regulation of 1-phosphatidyl-1D-myo-inositol 4,5-bisphosphate biosynthetic process, down regulation of 1-phosphatidyl-1D-myo-inositol 4,5-bisphosphate formation, down regulation of 1-phosphatidyl-1D-myo-inositol 4,5-bisphosphate synthesis, down-regulation of 1-phosphatidyl-1D-myo-inositol 4,5-bisphosphate anabolism, down-regulation of 1-phosphatidyl-1D-myo-inositol 4,5-bisphosphate biosynthesis, down-regulation of 1-phosphatidyl-1D-myo-inositol 4,5-bisphosphate biosynthetic process, down-regulation of 1-phosphatidyl-1D-myo-inositol 4,5-bisphosphate formation, down-regulation of 1-phosphatidyl-1D-myo-inositol 4,5-bisphosphate synthesis, downregulation of 1-phosphatidyl-1D-myo-inositol 4,5-bisphosphate anabolism, downregulation of 1-phosphatidyl-1D-myo-inositol 4,5-bisphosphate biosynthesis, downregulation of 1-phosphatidyl-1D-myo-inositol 4,5-bisphosphate biosynthetic process, downregulation of 1-phosphatidyl-1D-myo-inositol 4,5-bisphosphate formation, downregulation of 1-phosphatidyl-1D-myo-inositol 4,5-bisphosphate synthesis, negative regulation of 1-phosphatidyl-1D-myo-inositol 4,5-bisphosphate anabolism, negative regulation of 1-phosphatidyl-1D-myo-inositol 4,5-bisphosphate biosynthesis, negative regulation of 1-phosphatidyl-1D-myo-inositol 4,5-bisphosphate formation, negative regulation of 1-phosphatidyl-1D-myo-inositol 4,5-bisphosphate synthesis, inhibition of 1-phosphatidyl-1D-myo-inositol 4,5-bisphosphate anabolism, inhibition of 1-phosphatidyl-1D-myo-inositol 4,5-bisphosphate biosynthesis, inhibition of 1-phosphatidyl-1D-myo-inositol 4,5-bisphosphate biosynthetic process, inhibition of 1-phosphatidyl-1D-myo-inositol 4,5-bisphosphate formation, inhibition of 1-phosphatidyl-1D-myo-inositol 4,5-bisphosphate synthesis